{
  "gene_name": "NEDD4-binding protein 1",
  "term_id": "GO:0003729",
  "term_label": "mRNA binding",
  "gene_symbol": "N4BP1",
  "gene": "UniProtKB:O75113"
}